regulation of T cell chemotaxis [GO:0010819] (biological process) Subtypes: positive regulation of T cell chemotaxis [GO:0010820] Relationships: is a type of regulation of lymphocyte chemotaxis [GO:1901623]; is a type of GO:2000404; regulates GO:0010818 Sources: GOC:dph, GOC:tb Definition: Any process that modulates the rate, frequency or extent of T cell chemotaxis. T cell chemotaxis is the directed movement of a T cell in response to an external stimulus.